negative regulation of nucleotide metabolic process [GO:0045980] (biological process) Subtypes: negative regulation of nucleotide biosynthetic process [GO:0030809], negative regulation of nucleotide catabolic process [GO:0030812], negative regulation of purine nucleotide metabolic process [GO:1900543] Also known as: down regulation of nucleotide metabolic process, down-regulation of nucleotide metabolic process, downregulation of nucleotide metabolic process, negative regulation of nucleotide metabolism, inhibition of nucleotide metabolic process Sources: GOC:go_curators Definition: Any process that stops, prevents, or reduces the frequency, rate or extent of the chemical reactions and pathways involving nucleotides. Relationships: is a type of GO:0006140; is a type of negative regulation of nucleobase-containing compound metabolic process [GO:0045934]; is a type of GO:0045936; is_a negative regulation of small molecule metabolic process [GO:0062014]; RO_0002212 GO:0009117